2-succinyl-5-enolpyruvyl-6-hydroxy-3-cyclohexene-1-carboxylic-acid synthase activity [GO:0070204] (MF) Relationships: is a type of transketolase or transaldolase activity [GO:0016744] Sources: RHEA:25593 Definition: Catalysis of the reaction: 2-oxoglutarate + H+ + isochorismate = 5-enolpyruvoyl-6-hydroxy-2-succinyl-cyclohex-3-ene-1-carboxylate + CO2. Also known as: MenD, SEPHCHC synthase activity